{
  "term_id": "GO:0005634",
  "term_label": "nucleus",
  "gene_symbol": "ASCC3",
  "gene_name": "Activating signal cointegrator 1 complex subunit 3",
  "gene": "UniProtKB:Q8N3C0"
}